{
  "gene_name": "Heterogeneous nuclear ribonucleoprotein A3",
  "term_label": "mRNA 3'-UTR binding",
  "term_id": "GO:0003730",
  "gene": "UniProtKB:P51991",
  "gene_symbol": "HNRNPA3"
}